trans-activation response element binding [GO:1990970] (molecular function) Relationships: is a type of pre-miRNA binding [GO:0070883] Definition: Binding to a trans-activation response (TAR) element, a hairpin RNA structure located at the 5' end of all HIV-1 transcripts, and which is required for trans-activation of a viral promoter. Also known as: TAR binding References: PMID:25116364 Sources: GOC:PARL, GOC:bf, Wikipedia:Trans-activation_response_element_(TAR)